{
  "term_label": "Unknown biological process",
  "gene_symbol": "PXMP2",
  "gene_name": "Peroxisomal membrane protein 2",
  "term_id": "UNKNOWN:0002",
  "gene": "UniProtKB:Q9NR77"
}